nitric oxide biosynthetic process [GO:0006809] (biological process) Sources: GOC:ai Also known as: nitric oxide anabolism, nitric oxide biosynthesis, nitric oxide formation, nitric oxide synthesis Regulation: negatively regulated by negative regulation of nitric oxide biosynthetic process [GO:0045019]; regulated by regulation of nitric oxide biosynthetic process [GO:0045428]; positively regulated by positive regulation of nitric oxide biosynthetic process [GO:0045429] Definition: The chemical reactions and pathways resulting in the formation of nitric oxide, nitrogen monoxide (NO), a colorless gas only slightly soluble in water. Relationships: is a type of biosynthetic process [GO:0009058]; is a type of GO:0046209